{
  "gene": "UniProtKB:P41217",
  "gene_name": "OX-2 membrane glycoprotein",
  "term_label": "negative regulation of neuroinflammatory response",
  "term_id": "GO:0150079",
  "gene_symbol": "CD200"
}